{
  "term_label": "oligosaccharide metabolic process",
  "gene": "UniProtKB:P61647",
  "gene_symbol": "ST8SIA6",
  "gene_name": "Alpha-2,8-sialyltransferase 8F",
  "term_id": "GO:0009311"
}